tRNA (cytidine-3-)-methyltransferase activity [GO:0052735] (molecular function) Sources: RHEA:60908 Relationships: is a type of tRNA (cytidine) methyltransferase activity [GO:0016427] Also known as: S-adenosyl-L-methionine:tRNA (cytosine-3-)-methyltransferase activity, S-adenosyl-L-methionine:tRNA cytosine-3-methyltransferase activity, tRNA (cytosine 3)-methyltransferase activity, tRNA (cytosine-3-)-methyltransferase activity, tRNA cytosine 3-methyltransferase activity, tRNA cytosine-3-methyltransferase activity, transfer ribonucleate cytosine 3-methyltransferase activity Definition: Catalysis of the reaction: a cytidine in tRNA + S-adenosyl-L-methionine = an N3-methylcytidine in tRNA + H+ + S-adenosyl-L-homocysteine.